{
  "gene_symbol": "CMBL",
  "gene_name": "Carboxymethylenebutenolidase homolog",
  "term_label": "Unknown biological process",
  "gene": "UniProtKB:Q96DG6",
  "term_id": "UNKNOWN:0002"
}